{
  "gene_symbol": "TBCEL",
  "term_label": "alpha-tubulin binding",
  "gene_name": "Tubulin-specific chaperone cofactor E-like protein",
  "gene": "UniProtKB:Q5QJ74",
  "term_id": "GO:0043014"
}